{
  "gene_name": "S-adenosylmethionine decarboxylase proenzyme",
  "gene_symbol": "AMD1",
  "term_id": "GO:0005829",
  "term_label": "cytosol",
  "gene": "UniProtKB:P17707"
}